{
  "term_label": "plasma membrane",
  "gene": "UniProtKB:Q8NGZ6",
  "gene_symbol": "OR6F1",
  "term_id": "GO:0005886",
  "gene_name": "Olfactory receptor 6F1"
}